{
  "gene": "UniProtKB:P08908",
  "gene_name": "5-hydroxytryptamine receptor 1A",
  "term_label": "neurotransmitter receptor activity",
  "term_id": "GO:0030594",
  "gene_symbol": "HTR1A"
}